{
  "term_label": "endoplasmic reticulum to Golgi vesicle-mediated transport",
  "term_id": "GO:0006888",
  "gene_symbol": "CNIH4",
  "gene_name": "Protein cornichon homolog 4",
  "gene": "UniProtKB:Q9P003"
}